{
  "term_label": "nucleus",
  "gene_symbol": "PTEN",
  "gene_name": "Phosphatidylinositol 3,4,5-trisphosphate 3-phosphatase and dual-specificity protein phosphatase PTEN",
  "gene": "UniProtKB:P60484",
  "term_id": "GO:0005634"
}